{
  "term_label": "nucleosome",
  "term_id": "GO:0000786",
  "gene": "UniProtKB:P0C5Y9",
  "gene_symbol": "H2AB1",
  "gene_name": "Histone H2A-Bbd type 1"
}